{
  "gene_name": "Leukotriene A-4 hydrolase",
  "term_label": "aminopeptidase activity",
  "gene_symbol": "LTA4H",
  "gene": "UniProtKB:P09960",
  "term_id": "GO:0004177"
}